{
  "term_id": "GO:0006936",
  "gene": "UniProtKB:Q9NYL9",
  "term_label": "muscle contraction",
  "gene_symbol": "TMOD3",
  "gene_name": "Tropomodulin-3"
}